{
  "term_label": "Unknown molecular function",
  "gene_symbol": "SPCS1",
  "term_id": "UNKNOWN:0001",
  "gene_name": "Signal peptidase complex subunit 1",
  "gene": "UniProtKB:Q9Y6A9"
}